stomatal complex formation [GO:0010376] (biological process) Definition: The process that gives rise to the stomatal complex. This process pertains to the initial formation of a structure from unspecified parts. The stomatal complex is the stomatal guard cells and their associated epidermal cells. Relationships: is a type of GO:0048646; is part of stomatal complex morphogenesis [GO:0010103] References: PMID:17259259